{
  "gene_name": "Calcium-activated chloride channel regulator 1",
  "gene_symbol": "CLCA1",
  "gene": "UniProtKB:A8K7I4",
  "term_id": "GO:0005229",
  "term_label": "intracellularly calcium-gated chloride channel activity"
}